phosphatidate phosphatase activity [GO:0008195] (MF) References: PMID:25814022 Sources: GOC:pr, RHEA:27429 Definition: Catalysis of the reaction: a 1,2-diacylglycerol 3-phosphate + H2O = a 1,2-diacyl-sn-glycerol + phosphate. Also known as: phosphatidate phosphohydrolase activity, 3-sn-phosphatidate phosphohydrolase activity, acid phosphatidyl phosphatase activity, phosphatic acid phosphatase activity, phosphatic acid phosphohydrolase activity, phosphatidic acid phosphatase activity Relationships: is a type of lipid phosphatase activity [GO:0042577]